polyadenylation-dependent mRNA catabolic process [GO:0071047] (biological process) Subtypes: GO:0071042 Definition: The chemical reactions and pathways resulting in the breakdown of a messenger RNA (mRNA) molecule, initiated by the enzymatic addition of a sequence of adenylyl residues (polyadenylation) at the 3' end the target mRNA. Sources: GOC:dgf, GOC:krc Also known as: poly(A)-dependent mRNA catabolic process Relationships: is a type of GO:0006402; is a type of mRNA destabilization [GO:0061157]